{
  "term_label": "extracellular space",
  "gene_name": "Interleukin-7",
  "gene_symbol": "IL7",
  "term_id": "GO:0005615",
  "gene": "UniProtKB:P13232"
}